{
  "term_label": "mitotic spindle organization",
  "gene": "UniProtKB:Q15398",
  "gene_name": "Disks large-associated protein 5",
  "gene_symbol": "DLGAP5",
  "term_id": "GO:0007052"
}